5-formyluracil DNA N-glycosylase activity [GO:0034042] (molecular function) Also known as: 5-foU DNA N-glycosylase activity References: PMID:17641464 Sources: GOC:mah Relationships: is a type of oxidized pyrimidine nucleobase lesion DNA N-glycosylase activity [GO:0000703] Definition: Catalysis of the removal of 5-formyluracil bases by cleaving the N-C1' glycosidic bond between the oxidized pyrimidine and the deoxyribose sugar.